{
  "gene_name": "Histone deacetylase 3",
  "gene_symbol": "HDAC3",
  "term_label": "histone deacetylase complex",
  "gene": "UniProtKB:O15379",
  "term_id": "GO:0000118"
}